{
  "term_id": "GO:0007166",
  "gene_symbol": "CD80",
  "term_label": "cell surface receptor signaling pathway",
  "gene_name": "T-lymphocyte activation antigen CD80",
  "gene": "UniProtKB:P33681"
}